{
  "gene_symbol": "MT2A",
  "gene_name": "Metallothionein-2",
  "term_label": "cellular response to zinc ion",
  "gene": "UniProtKB:P02795",
  "term_id": "GO:0071294"
}